{
  "term_label": "Unknown cellular component",
  "gene_symbol": "GNB1L",
  "gene_name": "Guanine nucleotide-binding protein subunit beta-like protein 1",
  "gene": "UniProtKB:Q9BYB4",
  "term_id": "UNKNOWN:0003"
}